{
  "term_label": "lung development",
  "term_id": "GO:0030324",
  "gene_symbol": "FGF7",
  "gene_name": "Fibroblast growth factor 7",
  "gene": "UniProtKB:P21781"
}